{
  "gene_name": "T cell receptor gamma variable 5",
  "term_id": "UNKNOWN:0001",
  "gene": "UniProtKB:A0A0B4J1U4",
  "term_label": "Unknown molecular function",
  "gene_symbol": "TRGV5"
}